{
  "term_id": "UNKNOWN:0002",
  "gene_name": "Keratin-associated protein 9-3",
  "gene": "UniProtKB:Q9BYQ3",
  "term_label": "Unknown biological process",
  "gene_symbol": "KRTAP9-3"
}